coated membrane [GO:0048475] (cellular component) Definition: A single or double lipid bilayer with any of several different proteinaceous coats that can associate with membranes. Membrane coats include those formed by clathrin plus an adaptor complex, the COPI and COPII complexes. Sources: GOC:jid Relationships: is_a membrane [GO:0016020]